positive regulation of fertilization [GO:1905516] (biological process) Relationships: is a type of regulation of fertilization [GO:0080154]; is a type of positive regulation of reproductive process [GO:2000243]; positively regulates fertilization [GO:0009566] Also known as: positive regulation of syngamy, up regulation of fertilization, up regulation of syngamy, up-regulation of fertilization, up-regulation of syngamy, upregulation of fertilization, upregulation of syngamy, activation of fertilization, activation of syngamy Definition: Any process that activates or increases the frequency, rate or extent of fertilization. References: PMID:27564576 Sources: GOC:TermGenie, GOC:hbye, GO_REF:0000058